{
  "gene_symbol": "PLOD2",
  "term_label": "extracellular matrix",
  "term_id": "GO:0031012",
  "gene": "UniProtKB:O00469",
  "gene_name": "Procollagen-lysine,2-oxoglutarate 5-dioxygenase 2"
}